{
  "term_id": "GO:0045744",
  "gene_name": "Regulator of G-protein signaling 19",
  "gene": "UniProtKB:P49795",
  "gene_symbol": "RGS19",
  "term_label": "negative regulation of G protein-coupled receptor signaling pathway"
}